{
  "gene_name": "Trimethyllysine dioxygenase, mitochondrial",
  "gene": "UniProtKB:Q9NVH6",
  "term_label": "carnitine biosynthetic process",
  "gene_symbol": "TMLHE",
  "term_id": "GO:0045329"
}